{
  "gene_symbol": "IGHV2-5",
  "term_id": "UNKNOWN:0003",
  "gene": "UniProtKB:P01817",
  "gene_name": "Immunoglobulin heavy variable 2-5",
  "term_label": "Unknown cellular component"
}